 [go#goslim:prokaryote] Note: GO subset for prokaryotes